{
  "term_id": "GO:0030527",
  "gene": "UniProtKB:Q8IUE6",
  "gene_symbol": "H2AC21",
  "term_label": "structural constituent of chromatin",
  "gene_name": "Histone H2A type 2-B"
}